{
  "gene": "UniProtKB:A0MZ66",
  "gene_name": "Shootin-1",
  "gene_symbol": "SHTN1",
  "term_label": "axonal growth cone",
  "term_id": "GO:0044295"
}